{
  "gene": "UniProtKB:Q13237",
  "term_id": "GO:0007165",
  "term_label": "signal transduction",
  "gene_symbol": "PRKG2",
  "gene_name": "cGMP-dependent protein kinase 2"
}